platelet-derived growth factor receptor-alpha signaling pathway [GO:0035790] (biological process) References: PMID:10372961 Sources: GOC:bf, GOC:yaf Also known as: PDGF receptor-alpha signaling pathway, alphaPDGF receptor signaling pathway, platelet-derived growth factor receptor-alpha signalling pathway, PDGFR-alpha signaling pathway Subtypes: VEGF-activated platelet-derived growth factor receptor-alpha signaling pathway [GO:0038087] Definition: The series of molecular signals initiated a ligand binding to an alpha-type platelet-derived growth factor receptor (PDGFalpha) on the surface of a target cell, and ending with the regulation of a downstream cellular process, e.g. transcription. Relationships: is a type of platelet-derived growth factor receptor signaling pathway [GO:0048008] Regulation: RO_0002211 by regulation of platelet-derived growth factor receptor-alpha signaling pathway [GO:2000583]; RO_0002212 by negative regulation of platelet-derived growth factor receptor-alpha signaling pathway [GO:2000584]; positively regulated by positive regulation of platelet-derived growth factor receptor-alpha signaling pathway [GO:2000585]